{
  "gene": "UniProtKB:Q92994",
  "gene_symbol": "BRF1",
  "term_label": "transcription preinitiation complex",
  "term_id": "GO:0097550",
  "gene_name": "Transcription factor IIIB 90 kDa subunit"
}